negative regulation of anthocyanin catabolic process [GO:1900001] (biological process) Definition: Any process that stops, prevents or reduces the frequency, rate or extent of anthocyanin catabolic process. Also known as: down regulation of anthocyanin breakdown, down regulation of anthocyanin catabolism, down regulation of anthocyanin degradation, negative regulation of anthocyanin breakdown, negative regulation of anthocyanin catabolism, negative regulation of anthocyanin degradation, down regulation of anthocyanin catabolic process Sources: GOC:TermGenie Relationships: is a type of GO:0009895; is a type of negative regulation of anthocyanin metabolic process [GO:0031538]; is a type of regulation of anthocyanin catabolic process [GO:1900000]; negatively regulates anthocyanin-containing compound catabolic process [GO:0046284]